{
  "gene_symbol": "HSF5",
  "term_label": "nucleus",
  "gene_name": "Heat shock factor protein 5",
  "term_id": "GO:0005634",
  "gene": "UniProtKB:Q4G112"
}